{
  "term_id": "UNKNOWN:0001",
  "gene": "UniProtKB:Q96M60",
  "gene_name": "Protein FAM227B",
  "gene_symbol": "FAM227B",
  "term_label": "Unknown molecular function"
}